{
  "gene_symbol": "MYH9",
  "term_label": "actin filament binding",
  "term_id": "GO:0051015",
  "gene": "UniProtKB:P35579",
  "gene_name": "Myosin-9"
}